{
  "term_label": "positive regulation of G2/M transition of mitotic cell cycle",
  "term_id": "GO:0010971",
  "gene_symbol": "CDC25C",
  "gene_name": "M-phase inducer phosphatase 3",
  "gene": "UniProtKB:P30307"
}